{
  "gene_name": "Lysosomal cobalamin transport escort protein LMBD1",
  "gene": "UniProtKB:Q9NUN5",
  "term_id": "UNKNOWN:0001",
  "gene_symbol": "LMBRD1",
  "term_label": "Unknown molecular function"
}